{
  "term_id": "GO:0005829",
  "term_label": "cytosol",
  "gene": "UniProtKB:Q9BXW6",
  "gene_name": "Oxysterol-binding protein-related protein 1",
  "gene_symbol": "OSBPL1A"
}